{
  "gene": "UniProtKB:Q8NGA8",
  "gene_symbol": "OR4F17",
  "term_label": "Unknown cellular component",
  "term_id": "UNKNOWN:0003",
  "gene_name": "Olfactory receptor 4F17"
}